methanophenazine metabolic process [GO:1900629] (biological process) Subtypes: methanophenazine biosynthetic process [GO:1900630] Relationships: is a type of metabolic process [GO:0008152] Also known as: methanophenazine metabolism Sources: GOC:TermGenie, GOC:mengo_curators Definition: The chemical reactions and pathways involving methanophenazine.